{
  "term_label": "Unknown molecular function",
  "gene_name": "Formin-binding protein 1-like",
  "gene": "UniProtKB:Q5T0N5",
  "term_id": "UNKNOWN:0001",
  "gene_symbol": "FNBP1L"
}